{
  "term_id": "GO:0005829",
  "term_label": "cytosol",
  "gene": "UniProtKB:Q00994",
  "gene_name": "Protein BEX3",
  "gene_symbol": "BEX3"
}